GroEL-GroES complex [GO:1990220] (cellular component) Relationships: is a type of chaperonin ATPase complex [GO:0016465] Definition: Bacterial chaperonin complex consisting of a heptameric 10kDa chaperonin subunit GroES and a tetradecameric (2x7) 60kDa chaperonin subunit GroEL. The 60kDa subunit possesses ATPase activity while the holo-enzyme is responsible for the correct folding of proteins. References: PMID:15313620 Sources: GOC:bhm Also known as: bacterial chaperonin ATPase complex, bacterial chaperonin complex